{
  "term_label": "plasma membrane",
  "gene": "UniProtKB:Q7LBE3",
  "gene_symbol": "SLC26A9",
  "gene_name": "Solute carrier family 26 member 9",
  "term_id": "GO:0005886"
}